{
  "term_id": "GO:0006509",
  "gene_name": "Beta-secretase 2",
  "gene_symbol": "BACE2",
  "gene": "UniProtKB:Q9Y5Z0",
  "term_label": "membrane protein ectodomain proteolysis"
}